positive regulation of plasmatocyte differentiation [GO:0045615] (biological process) Definition: Any process that activates or increases the frequency, rate or extent of plasmatocyte differentiation. Also known as: up regulation of plasmatocyte differentiation, up-regulation of plasmatocyte differentiation, upregulation of plasmatocyte differentiation, activation of plasmatocyte differentiation, stimulation of plasmatocyte differentiation Sources: GOC:go_curators Relationships: is a type of positive regulation of hemocyte differentiation [GO:0045612]; is a type of regulation of plasmatocyte differentiation [GO:0045613]; positively regulates plasmatocyte differentiation [GO:0042387]